{
  "gene_name": "Protein FAM32A",
  "term_id": "UNKNOWN:0002",
  "gene_symbol": "FAM32A",
  "gene": "UniProtKB:Q9Y421",
  "term_label": "Unknown biological process"
}